gamma-delta T cell activation involved in immune response [GO:0002290] (biological process) Definition: The change in morphology and behavior of a gamma-delta T cell resulting from exposure to a mitogen, cytokine, chemokine, cellular ligand, or an antigen for which it is specific, leading to the initiation or perpetuation of an immune response. References: PMID:8717523 Sources: GOC:add Also known as: gamma-delta T cell activation during immune response, gamma-delta T lymphocyte activation during immune response, gamma-delta T-cell activation during immune response, gamma-delta T-lymphocyte activation during immune response Relationships: is a type of T cell activation involved in immune response [GO:0002286]; is_a GO:0046629 Subtypes: gamma-delta T cell differentiation involved in immune response [GO:0002303], gamma-delta T cell proliferation involved in immune response [GO:0002311] Regulation: regulated by GO:2001191; negatively regulated by GO:2001192; positively regulated by positive regulation of gamma-delta T cell activation involved in immune response [GO:2001193]